{
  "gene_name": "Olfactory receptor 4N5",
  "term_label": "Unknown biological process",
  "term_id": "UNKNOWN:0002",
  "gene_symbol": "OR4N5",
  "gene": "UniProtKB:Q8IXE1"
}